cortisol dehydrogenase (NADP+) activity [GO:0102196] (molecular function) Definition: Catalysis of the reaction: cortisol + NADP+ = cortisone + NADPH + H+. Relationships: is a type of GO:0070524 References: PMID:16216911 Sources: RHEA:68616